regulation of muscle atrophy [GO:0014735] (biological process) Definition: Any process that modulates the frequency, rate or extent of muscle atrophy. Sources: GOC:mtg_muscle Subtypes: negative regulation of muscle atrophy [GO:0014736], positive regulation of muscle atrophy [GO:0014737] Relationships: is a type of GO:0043502; regulates muscle atrophy [GO:0014889]